negative regulation of vulval development [GO:0040027] (biological process) Relationships: is a type of regulation of vulval development [GO:0040028]; is a type of negative regulation of nematode larval development [GO:0061064]; negatively regulates GO:0040025 Definition: Any process that stops, prevents, or reduces the frequency, rate or extent of development of the vulva. Vulval development is the process whose specific outcome is the progression of the egg-laying organ of female and hermaphrodite nematodes over time, from its formation to the mature structure. In nematodes, the vulva is formed from ventral epidermal cells during larval stages to give rise to a fully formed vulva in the adult. Also known as: down regulation of vulval development, down-regulation of vulval development, downregulation of vulval development, inhibition of vulval development Sources: GOC:ems, GOC:kmv